AGU codon-amino acid adaptor activity [GO:0033445] (molecular function) Note: Note that in the standard genetic code, AGT codes for serine. Sources: GOC:mah Relationships: is a type of GO:0030533 Also known as: AGT codon-amino acid adaptor activity, serine tRNA Definition: A triplet codon-amino acid adaptor activity that recognizes an AGU codon.